{
  "gene_symbol": "CHORDC1",
  "gene": "UniProtKB:Q9UHD1",
  "term_label": "centrosome duplication",
  "gene_name": "Cysteine and histidine-rich domain-containing protein 1",
  "term_id": "GO:0051298"
}